proteolysis by cytosolic proteases associated with antigen processing and presentation [GO:0002203] (biological process) References: PMID:15224092, PMID:15771591 Sources: GOC:add, ISBN:0781735149 Note: Note that a separate term covers proteolysis by the proteasome complex (proteasomal proteolysis associated with antigen processing and presentation ; GO:0002497). Definition: The hydrolysis of a peptide bond or bonds within a protein by cytosolic resident proteases during antigen processing and presentation. Relationships: is a type of proteolysis associated with antigen processing and presentation [GO:0002496]